{
  "term_id": "UNKNOWN:0002",
  "gene": "UniProtKB:A0A1B0GTH9",
  "gene_name": "Zinc finger protein 474",
  "gene_symbol": "LOC100505841",
  "term_label": "Unknown biological process"
}